{
  "term_id": "GO:0005739",
  "gene_name": "Activator of apoptosis harakiri",
  "term_label": "mitochondrion",
  "gene": "UniProtKB:O00198",
  "gene_symbol": "HRK"
}